{
  "term_id": "GO:0007186",
  "gene": "UniProtKB:Q15726",
  "gene_name": "Metastasis-suppressor KiSS-1",
  "term_label": "G protein-coupled receptor signaling pathway",
  "gene_symbol": "KISS1"
}